{
  "term_id": "GO:0070822",
  "gene_symbol": "PHF12",
  "gene": "UniProtKB:Q96QT6",
  "term_label": "Sin3-type complex",
  "gene_name": "PHD finger protein 12"
}